{
  "gene": "UniProtKB:Q9Y5S9",
  "gene_symbol": "RBM8A",
  "term_label": "RNA splicing",
  "gene_name": "RNA-binding protein 8A",
  "term_id": "GO:0008380"
}